{
  "term_label": "Unknown molecular function",
  "gene_name": "Golgin subfamily A member 6-like protein 2",
  "term_id": "UNKNOWN:0001",
  "gene": "UniProtKB:Q8N9W4",
  "gene_symbol": "GOLGA6L2"
}